{
  "gene_symbol": "LAX1",
  "term_id": "UNKNOWN:0001",
  "gene": "UniProtKB:Q8IWV1",
  "term_label": "Unknown molecular function",
  "gene_name": "Lymphocyte transmembrane adapter 1"
}